{
  "gene_name": "Cyclin-dependent kinase 5",
  "gene_symbol": "CDK5",
  "term_id": "GO:0005737",
  "term_label": "cytoplasm",
  "gene": "UniProtKB:Q00535"
}